detection of UV [GO:0009589] (biological process) Sources: GOC:dos, GOC:go_curators, GOC:hb, ISBN:0198506732 Also known as: detection of UV light stimulus, detection of UV radiation stimulus, detection of ultraviolet light stimulus, detection of ultraviolet radiation stimulus, perception of UV Subtypes: GO:0007604 Relationships: is a type of response to UV [GO:0009411]; is a type of detection of light stimulus [GO:0009583] Definition: The series of events in which an ultraviolet radiation (UV light) stimulus is received and converted into a molecular signal. Ultraviolet radiation is electromagnetic radiation with a wavelength in the range of 10 to 380 nanometers.